cell wall repair [GO:0071433] (biological process) Sources: GOC:mah, GOC:vw Relationships: is a type of cell wall organization [GO:0071555] Definition: A process of cell wall organization that results in the restoration of the cell wall following damage.